amylo-alpha-1,6-glucosidase activity [GO:0004135] (molecular function) Sources: EC:3.2.1.33 Definition: Catalysis of the hydrolysis of (1->6)-alpha-D-glucosidic branch linkages in glycogen phosphorylase limit dextrin. Limit dextrin is the highly branched core that remains after exhaustive treatment of glycogen with glycogen phosphorylase. It is formed because these enzymes cannot hydrolyze the (1->6) glycosidic linkages present. Relationships: is a type of alpha-glucosidase activity [GO:0090599] Also known as: amylo-1,6-glucosidase activity, amylopectin 1,6-glucosidase activity, dextrin 6-alpha-D-glucosidase activity, dextrin-1,6-glucosidase activity, glycogen phosphorylase-limit dextrin alpha-1,6-glucohydrolase activity